{
  "gene_name": "Protein furry homolog",
  "gene": "UniProtKB:Q5TBA9",
  "term_label": "neuron projection development",
  "term_id": "GO:0031175",
  "gene_symbol": "FRY"
}